{
  "gene_symbol": "TEX13B",
  "gene_name": "Testis-expressed protein 13B",
  "term_label": "mRNA binding",
  "gene": "UniProtKB:Q9BXU2",
  "term_id": "GO:0003729"
}